amyloid-beta metabolic process [GO:0050435] (biological process) Also known as: amyloid-beta metabolism, beta-amyloid metabolic process, beta-amyloid metabolism Sources: GOC:ai Relationships: is a type of amide metabolic process [GO:0043603] Definition: The chemical reactions and pathways involving amyloid-beta, a glycoprotein associated with Alzheimer's disease, and its precursor, amyloid precursor protein (APP). Subtypes: amyloid-beta formation [GO:0034205], amyloid-beta clearance by cellular catabolic process [GO:0150094]